{
  "term_id": "GO:0006421",
  "gene_symbol": "NARS2",
  "gene": "UniProtKB:Q96I59",
  "gene_name": "Probable asparagine--tRNA ligase, mitochondrial",
  "term_label": "asparaginyl-tRNA aminoacylation"
}